{
  "term_label": "SNAP receptor activity",
  "gene_symbol": "STX5",
  "term_id": "GO:0005484",
  "gene": "UniProtKB:Q13190",
  "gene_name": "Syntaxin-5"
}